Toll-like receptor 1-Toll-like receptor 2 protein complex [GO:0035354] (cellular component) Definition: A heterodimeric protein complex containing Toll-like receptor 1 (TLR1) and Toll-like receptor 2 (TLR2). References: PMID:17889651, PMID:21481769 Sources: GOC:add, GOC:signaling Also known as: TLR1-TLR2 protein complex, TLR1:TLR2 complex, TLR2:TLR1 heterodimer, toll-like receptor TLR1:TLR2 heterodimeric complex Relationships: is a type of plasma membrane signaling receptor complex [GO:0098802]